{
  "term_id": "GO:0006886",
  "term_label": "intracellular protein transport",
  "gene": "UniProtKB:Q16623",
  "gene_name": "Syntaxin-1A",
  "gene_symbol": "STX1A"
}